{
  "gene_name": "Guanine nucleotide-binding protein G(o) subunit alpha",
  "gene_symbol": "GNAO1",
  "gene": "UniProtKB:P09471",
  "term_id": "GO:0031821",
  "term_label": "G protein-coupled serotonin receptor binding"
}